{
  "gene": "UniProtKB:Q9NVV0",
  "term_id": "GO:0071805",
  "term_label": "potassium ion transmembrane transport",
  "gene_symbol": "TMEM38B",
  "gene_name": "Trimeric intracellular cation channel type B"
}